positive regulation of neuroblast migration [GO:0061854] (biological process) Definition: Any process that activates or increases the frequency, rate or extent of neuroblast migration. References: PMID:23149556 Relationships: is a type of positive regulation of cell migration [GO:0030335]; is a type of regulation of neuroblast migration [GO:0061853]; positively regulates neuroblast migration [GO:0097402]